{
  "gene_symbol": "CCDC102B",
  "gene_name": "Coiled-coil domain-containing protein 102B",
  "term_id": "UNKNOWN:0003",
  "gene": "UniProtKB:Q68D86",
  "term_label": "Unknown cellular component"
}